{
  "term_label": "dynactin complex",
  "gene_name": "Alpha-centractin",
  "term_id": "GO:0005869",
  "gene_symbol": "ACTR1A",
  "gene": "UniProtKB:P61163"
}